{
  "gene_name": "Small ubiquitin-related modifier 2",
  "term_id": "GO:0016925",
  "term_label": "protein sumoylation",
  "gene": "UniProtKB:P61956",
  "gene_symbol": "SUMO2"
}